angiotensin type I receptor activity [GO:0001596] (molecular function) References: PMID:10977869 Sources: GOC:mah Relationships: is a type of angiotensin receptor activity [GO:0001595]; is part of phospholipase C-activating angiotensin-activated signaling pathway [GO:0086097] Definition: An angiotensin receptor activity that acts via Gq-mediated activation of phospholipase C followed by phosphoinositide hydrolysis and Ca2+ signaling, and may act via additional signaling mechanisms. Also known as: PLC-activating angiotensin receptor activity